establishment of body hair or bristle planar orientation [GO:0048104] (BP) Definition: Orientation of hairs or sensory bristles that cover the body surface of an adult, such that they all point in a uniform direction along the plane of the epithelium from which they project. Relationships: is a type of establishment of planar polarity [GO:0001736] Subtypes: establishment of body hair planar orientation [GO:0048105], establishment of thoracic bristle planar orientation [GO:0048106] Sources: GOC:ascb_2009, GOC:dph, GOC:jid, GOC:tb